{
  "gene_symbol": "POTEJ",
  "gene_name": "POTE ankyrin domain family member J",
  "term_label": "cell motility",
  "gene": "UniProtKB:P0CG39",
  "term_id": "GO:0048870"
}